ribose 1,5-bisphosphate phosphokinase activity [GO:0033863] (molecular function) Relationships: is a type of phosphotransferase activity, phosphate group as acceptor [GO:0016776]; is a type of carbohydrate kinase activity [GO:0019200] Definition: Catalysis of the reaction: D-ribose 1,5-diphosphate + ATP = 5-phospho-alpha-D-ribose 1-diphosphate + ADP + H+. Sources: EC:2.7.4.23, RHEA:20109 Also known as: ATP:ribose-1,5-bisphosphate phosphotransferase activity, PhnN, ribose 1,5-bisphosphokinase activity